intracellular nucleoside transport [GO:0015859] (biological process) Relationships: is a type of GO:0015858; is a type of intracellular transport [GO:0046907] Sources: GOC:ai Definition: The directed movement of a nucleoside, a nucleobase linked to either beta-D-ribofuranose (ribonucleoside) or 2-deoxy-beta-D-ribofuranose, (a deoxyribonucleotide), within a cell.